{
  "term_label": "regulation of gene expression",
  "term_id": "GO:0010468",
  "gene_symbol": "KDM4D",
  "gene_name": "Lysine-specific demethylase 4D",
  "gene": "UniProtKB:Q6B0I6"
}